{
  "gene_symbol": "CLEC11A",
  "term_label": "growth factor activity",
  "term_id": "GO:0008083",
  "gene": "UniProtKB:Q9Y240",
  "gene_name": "C-type lectin domain family 11 member A"
}